{
  "gene": "UniProtKB:Q3SXP7",
  "term_id": "UNKNOWN:0003",
  "gene_symbol": "SHISAL1",
  "term_label": "Unknown cellular component",
  "gene_name": "Protein shisa-like-1"
}